GDP metabolic process [GO:0046710] (biological process) Also known as: GDP metabolism Subtypes: GO:0046711, GDP catabolic process [GO:0046712] Definition: The chemical reactions and pathways involving GDP, guanosine 5'-diphosphate. Sources: GOC:ai Relationships: is a type of purine ribonucleotide metabolic process [GO:0009150]; is a type of purine ribonucleoside diphosphate metabolic process [GO:0009179]